{
  "term_id": "UNKNOWN:0001",
  "gene_name": "Actin-binding Rho-activating protein",
  "gene": "UniProtKB:Q8N0Z2",
  "term_label": "Unknown molecular function",
  "gene_symbol": "ABRA"
}